{
  "term_id": "GO:0060041",
  "gene": "UniProtKB:O43316",
  "term_label": "retina development in camera-type eye",
  "gene_name": "Paired box protein Pax-4",
  "gene_symbol": "PAX4"
}